{
  "term_label": "peroxisome",
  "gene_name": "Acyl-coenzyme A oxidase-like protein",
  "gene": "UniProtKB:Q9NUZ1",
  "gene_symbol": "ACOXL",
  "term_id": "GO:0005777"
}